{
  "gene_name": "Centrin-3",
  "gene_symbol": "CETN3",
  "term_id": "GO:0005815",
  "term_label": "microtubule organizing center",
  "gene": "UniProtKB:O15182"
}